{
  "gene_name": "Endoribonuclease Dicer",
  "gene": "UniProtKB:Q9UPY3",
  "term_id": "GO:0004525",
  "term_label": "ribonuclease III activity",
  "gene_symbol": "DICER1"
}